cardiac septum cell differentiation [GO:0003292] (biological process) Sources: GOC:mtg_heart Relationships: is a type of cardiocyte differentiation [GO:0035051]; is part of cardiac septum development [GO:0003279] Definition: The process in which an endocardial cushion cell becomes a cell of a cardiac septum. Subtypes: atrioventricular node cell differentiation [GO:0060922]